positive regulation of odontoblast differentiation [GO:1901331] (biological process) Definition: Any process that activates or increases the frequency, rate or extent of odontoblast differentiation. Relationships: is a type of regulation of odontoblast differentiation [GO:1901329]; is a type of GO:1902913; positively regulates odontoblast differentiation [GO:0071895] Sources: GOC:TermGenie Also known as: up regulation of odontoblast differentiation, up-regulation of odontoblast differentiation, upregulation of odontoblast differentiation, activation of odontoblast differentiation